{
  "gene_name": "Mediator of RNA polymerase II transcription subunit 24",
  "term_label": "transcription coregulator activity",
  "gene": "UniProtKB:O75448",
  "gene_symbol": "MED24",
  "term_id": "GO:0003712"
}